{
  "gene_symbol": "ZFAT",
  "gene": "UniProtKB:Q9P243",
  "gene_name": "Zinc finger protein ZFAT",
  "term_label": "RNA polymerase II cis-regulatory region sequence-specific DNA binding",
  "term_id": "GO:0000978"
}